{
  "term_label": "exon-exon junction complex",
  "term_id": "GO:0035145",
  "gene_symbol": "RBM8A",
  "gene_name": "RNA-binding protein 8A",
  "gene": "UniProtKB:Q9Y5S9"
}